{
  "term_id": "GO:0005634",
  "gene_name": "Fibroblast growth factor 2",
  "gene": "UniProtKB:P09038",
  "term_label": "nucleus",
  "gene_symbol": "FGF2"
}